lateral line system development [GO:0048925] (biological process) Definition: The process whose specific outcome is the progression of the lateral line system over time, from its formation to the mature structure. The lateral line system is a network of sensory organs (neuromasts) and lateral line nerves located superficially on the skin or just under the skin in fluid-filled canals on the head and body of all fishes and most amphibians. The lateral line system develops from cranial ectodermal placodes situated between the eye and ear. Sources: GOC:dgh, ISBN:0125296509 Relationships: is a type of GO:0048880 Subtypes: mechanosensory lateral line system development [GO:0048881], anterior lateral line system development [GO:0048898], posterior lateral line system development [GO:0048915], GO:0048926